{
  "gene": "UniProtKB:Q9BYH8",
  "gene_name": "NF-kappa-B inhibitor zeta",
  "gene_symbol": "NFKBIZ",
  "term_label": "Unknown molecular function",
  "term_id": "UNKNOWN:0001"
}